{
  "gene_name": "Lysosomal acid lipase_cholesteryl ester hydrolase",
  "gene_symbol": "LIPA",
  "gene": "UniProtKB:P38571",
  "term_id": "GO:0016125",
  "term_label": "sterol metabolic process"
}